{
  "gene": "UniProtKB:P48378",
  "gene_name": "DNA-binding protein RFX2",
  "term_label": "regulation of transcription by RNA polymerase II",
  "term_id": "GO:0006357",
  "gene_symbol": "RFX2"
}